iron ion import across cell outer membrane [GO:0098706] (biological process) Definition: The directed movement of iron ions from outside of a cell, across the cell outer membrane and into the periplasmic space. Relationships: is a type of iron ion transmembrane transport [GO:0034755] References: PMID:23192658 Sources: GOC:mah Also known as: ferric iron transmembrane transport, ferric ion import into cell, ferric iron import into cell, ferric iron import across cell outer membrane, high affinity ferric iron transport, high-affinity ferric iron transmembrane transport